{
  "gene": "UniProtKB:Q8WW35",
  "term_id": "GO:0007018",
  "gene_name": "Dynein light chain Tctex-type protein 2B",
  "gene_symbol": "DYNLT2B",
  "term_label": "microtubule-based movement"
}